purine ribonucleotide metabolic process [GO:0009150] (biological process) Also known as: purine ribonucleotide metabolism Subtypes: purine ribonucleotide biosynthetic process [GO:0009152], purine ribonucleotide catabolic process [GO:0009154], purine ribonucleotide interconversion [GO:0015951], GO:0015969, guanosine pentaphosphate metabolic process [GO:0015972], ADP metabolic process [GO:0046031], AMP metabolic process [GO:0046033], ATP metabolic process [GO:0046034], GMP metabolic process [GO:0046037], GO:0046039, IMP metabolic process [GO:0046040], ITP metabolic process [GO:0046041], GO:0046058, cGMP metabolic process [GO:0046068], IDP metabolic process [GO:0046707], GDP metabolic process [GO:0046710], 3'-phosphoadenosine 5'-phosphosulfate metabolic process [GO:0050427], XMP metabolic process [GO:0097292] Definition: The chemical reactions and pathways involving a purine ribonucleotide, a compound consisting of ribonucleoside (a purine base linked to a ribose sugar) esterified with a phosphate group at either the 3' or 5'-hydroxyl group of the sugar. Sources: GOC:go_curators, ISBN:0198506732 Relationships: is a type of purine nucleotide metabolic process [GO:0006163]; is a type of GO:0009259